genitalia morphogenesis [GO:0035112] (biological process) Definition: The process in which the anatomical structures of genitalia are generated and organized. The genitalia are the organs of reproduction or generation, external and internal. Sources: GOC:bf Also known as: genital morphogenesis Subtypes: embryonic genitalia morphogenesis [GO:0030538], post-embryonic genitalia morphogenesis [GO:0035126], internal genitalia morphogenesis [GO:0035260], GO:0035261, female genitalia morphogenesis [GO:0048807], male genitalia morphogenesis [GO:0048808] Relationships: is a type of developmental process involved in reproduction [GO:0003006]; is a type of animal organ morphogenesis [GO:0009887]; is part of GO:0048806